{
  "term_id": "GO:0033204",
  "gene_symbol": "RPP14",
  "term_label": "ribonuclease P RNA binding",
  "gene_name": "Ribonuclease P protein subunit p14",
  "gene": "UniProtKB:O95059"
}